{
  "gene_symbol": "RCAN3",
  "term_id": "GO:0005634",
  "gene_name": "Calcipressin-3",
  "gene": "UniProtKB:Q9UKA8",
  "term_label": "nucleus"
}